{
  "gene": "UniProtKB:Q9BZW4",
  "gene_symbol": "TM6SF2",
  "gene_name": "Transmembrane 6 superfamily member 2",
  "term_label": "endoplasmic reticulum-Golgi intermediate compartment membrane",
  "term_id": "GO:0033116"
}